{
  "term_id": "GO:0030032",
  "gene": "UniProtKB:O14639",
  "gene_symbol": "ABLIM1",
  "term_label": "lamellipodium assembly",
  "gene_name": "Actin-binding LIM protein 1"
}